corrin biosynthetic process [GO:0046140] (biological process) Relationships: is a type of tetrapyrrole biosynthetic process [GO:0033014] Also known as: corrin anabolism, corrin biosynthesis, corrin formation, corrin synthesis Sources: GOC:ai Definition: The chemical reactions and pathways resulting in the formation of corrin, C19H22N4, the fundamental heterocyclic skeleton of the corrinoids. It consists of four reduced pyrrole rings joined into a macrocyclic ring. Corrin is the core of the vitamin B12 molecule.